{
  "gene": "UniProtKB:A8MVU1",
  "term_label": "respiratory burst",
  "term_id": "GO:0045730",
  "gene_name": "Putative neutrophil cytosol factor 1C",
  "gene_symbol": "NCF1C"
}